mesenchymal stem cell differentiation involved in nephron morphogenesis [GO:0072037] (biological process) Sources: GOC:mtg_kidney_jan10 Definition: The process in which a relatively unspecialized cell acquires specialized features of a mesenchymal stem cell that contributes to the shaping of a nephron. A mesenchymal stem cell is a cell that retains the ability to divide and proliferate throughout life to provide progenitor cells that can differentiate into specialized mesenchymal cells. Subtypes: GO:0061239, mesenchymal stem cell differentiation involved in metanephric nephron morphogenesis [GO:0072281] Relationships: is a type of GO:0061005; is a type of mesenchymal stem cell differentiation [GO:0072497]; is part of nephron morphogenesis [GO:0072028]